{
  "term_id": "GO:0005793",
  "gene": "UniProtKB:O15260",
  "gene_symbol": "SURF4",
  "term_label": "endoplasmic reticulum-Golgi intermediate compartment",
  "gene_name": "Surfeit locus protein 4"
}